{
  "gene_symbol": "ZNF280D",
  "gene": "UniProtKB:Q6N043",
  "gene_name": "Zinc finger protein 280D",
  "term_id": "GO:0000978",
  "term_label": "RNA polymerase II cis-regulatory region sequence-specific DNA binding"
}